{
  "term_label": "hormone-mediated signaling pathway",
  "term_id": "GO:0009755",
  "gene": "UniProtKB:P22888",
  "gene_name": "Lutropin-choriogonadotropic hormone receptor",
  "gene_symbol": "LHCGR"
}